{
  "gene_name": "Hematopoietically-expressed homeobox protein HHEX",
  "gene": "UniProtKB:Q03014",
  "term_label": "cell differentiation",
  "gene_symbol": "HHEX",
  "term_id": "GO:0030154"
}